{
  "gene": "UniProtKB:Q5FWF4",
  "gene_name": "DNA annealing helicase and endonuclease ZRANB3",
  "gene_symbol": "ZRANB3",
  "term_id": "GO:0006281",
  "term_label": "DNA repair"
}